negative regulation of central B cell anergy [GO:0002915] (biological process) Sources: GOC:add Definition: Any process that stops, prevents, or reduces the frequency, rate, or extent of central B cell anergy. Relationships: is a type of negative regulation of B cell anergy [GO:0002671]; is a type of negative regulation of central B cell tolerance induction [GO:0002896]; is_a GO:0002914; is a type of negative regulation of B cell differentiation [GO:0045578]; negatively regulates central B cell anergy [GO:0002341] Also known as: down regulation of central B cell anergy, down-regulation of central B cell anergy, downregulation of central B cell anergy, inhibition of central B cell anergy